{
  "term_label": "tubulin binding",
  "gene": "UniProtKB:P61601",
  "gene_symbol": "NCALD",
  "term_id": "GO:0015631",
  "gene_name": "Neurocalcin-delta"
}